{
  "gene": "UniProtKB:P08172",
  "term_label": "G protein-coupled acetylcholine receptor activity",
  "gene_name": "Muscarinic acetylcholine receptor M2",
  "gene_symbol": "CHRM2",
  "term_id": "GO:0016907"
}